{
  "term_id": "GO:0005737",
  "gene_name": "Cysteine protease ATG4D",
  "term_label": "cytoplasm",
  "gene": "UniProtKB:Q86TL0",
  "gene_symbol": "ATG4D"
}